{
  "term_label": "Unknown biological process",
  "term_id": "UNKNOWN:0002",
  "gene": "UniProtKB:Q6P1R3",
  "gene_symbol": "MSANTD2",
  "gene_name": "Myb_SANT-like DNA-binding domain-containing protein 2"
}